{
  "term_label": "arachidonate 15-lipoxygenase activity",
  "gene_name": "Polyunsaturated fatty acid lipoxygenase ALOX15B",
  "term_id": "GO:0050473",
  "gene_symbol": "ALOX15B",
  "gene": "UniProtKB:O15296"
}